{
  "gene_name": "Forkhead box protein P1",
  "gene_symbol": "FOXP1",
  "gene": "UniProtKB:Q9H334",
  "term_label": "RNA polymerase II cis-regulatory region sequence-specific DNA binding",
  "term_id": "GO:0000978"
}